{
  "gene_symbol": "ACOT13",
  "term_label": "Unknown cellular component",
  "gene": "UniProtKB:Q9NPJ3",
  "term_id": "UNKNOWN:0003",
  "gene_name": "Acyl-coenzyme A thioesterase 13"
}